terminal cisterna [GO:0014802] (CC) Relationships: is_a endoplasmic reticulum subcompartment [GO:0098827]; is part of sarcoplasmic reticulum [GO:0016529] Definition: The portion of sarcoplasmic reticulum devoted to calcium ion storage and calcium ion release. Sources: GOC:mtg_muscle